{
  "gene_name": "Double homeobox protein 4-like protein 5",
  "term_id": "GO:0005634",
  "gene_symbol": "DUX4L5",
  "gene": "UniProtKB:P0CJ88",
  "term_label": "nucleus"
}